{
  "gene_name": "Neuropilin-1",
  "term_id": "GO:0002040",
  "gene": "UniProtKB:O14786",
  "term_label": "sprouting angiogenesis",
  "gene_symbol": "NRP1"
}